muscle cell postsynaptic specialization [GO:0097482] (cellular component) Relationships: is a type of postsynaptic specialization [GO:0099572]; is part of postsynapse of neuromuscular junction [GO:0098975] Also known as: muscle cell postsynaptic density, muscle fiber postsynaptic density Definition: A postsynaptic specialization that is part of a neuromuscular junction. Sources: GOC:pr